quinoline 2-oxidoreductase activity [GO:0018523] (molecular function) Sources: EC:1.3.99.17 Relationships: is a type of oxidoreductase activity, acting on the CH-CH group of donors [GO:0016627] Definition: Catalysis of the reaction: quinoline + acceptor + H2O = isoquinolin-1(2H)-one + reduced acceptor. Also known as: quinoline:acceptor 2-oxidoreductase (hydroxylating)